{
  "term_label": "precatalytic spliceosome",
  "gene": "UniProtKB:P62314",
  "gene_symbol": "SNRPD1",
  "gene_name": "Small nuclear ribonucleoprotein Sm D1",
  "term_id": "GO:0071011"
}